negative regulation of prolactin signaling pathway [GO:1902212] (biological process) References: PMID:11773439 Sources: GOC:TermGenie Also known as: down regulation of PRL signaling pathway, down regulation of prolactin signaling pathway, down regulation of prolactin-mediated signaling pathway, down-regulation of PRL signaling pathway, down-regulation of prolactin signaling pathway, down-regulation of prolactin-mediated signaling pathway, downregulation of PRL signaling pathway, downregulation of prolactin signaling pathway, downregulation of prolactin-mediated signaling pathway, negative regulation of PRL signaling pathway, negative regulation of prolactin-mediated signaling pathway, inhibition of PRL signaling pathway, inhibition of prolactin signaling pathway, inhibition of prolactin-mediated signaling pathway Relationships: is a type of negative regulation of cytokine-mediated signaling pathway [GO:0001960]; is a type of regulation of prolactin signaling pathway [GO:1902211]; negatively regulates prolactin signaling pathway [GO:0038161] Definition: Any process that stops, prevents or reduces the frequency, rate or extent of prolactin signaling pathway.